{
  "term_id": "GO:0006120",
  "gene": "UniProtKB:Q9Y375",
  "gene_symbol": "NDUFAF1",
  "term_label": "mitochondrial electron transport, NADH to ubiquinone",
  "gene_name": "Complex I intermediate-associated protein 30, mitochondrial"
}